{
  "term_label": "cytoplasm",
  "gene": "UniProtKB:P49802",
  "term_id": "GO:0005737",
  "gene_name": "Regulator of G-protein signaling 7",
  "gene_symbol": "RGS7"
}